{
  "term_label": "Unknown molecular function",
  "gene_symbol": "RSRP1",
  "gene_name": "Arginine_serine-rich protein 1",
  "gene": "UniProtKB:Q9BUV0",
  "term_id": "UNKNOWN:0001"
}